{
  "term_id": "GO:0003743",
  "term_label": "translation initiation factor activity",
  "gene": "UniProtKB:A6NMX2",
  "gene_symbol": "EIF4E1B",
  "gene_name": "Eukaryotic translation initiation factor 4E type 1B"
}